regulation of toll-like receptor 15 signaling pathway [GO:2000440] (biological process) Also known as: regulation of TLR15 signaling pathway, regulation of toll-like receptor 15 signalling pathway Relationships: is a type of regulation of pattern recognition receptor signaling pathway [GO:0062207]; regulates toll-like receptor 15 signaling pathway [GO:0035681] Definition: Any process that modulates the frequency, rate or extent of toll-like receptor 15 signaling pathway. Sources: GOC:obol Subtypes: GO:2000441, GO:2000442